{
  "term_label": "Unknown molecular function",
  "gene_name": "Beta-catenin-like protein 1",
  "gene_symbol": "CTNNBL1",
  "gene": "UniProtKB:Q8WYA6",
  "term_id": "UNKNOWN:0001"
}